{
  "term_id": "GO:0005886",
  "term_label": "plasma membrane",
  "gene_name": "Rho GTPase-activating protein 27",
  "gene": "UniProtKB:Q6ZUM4",
  "gene_symbol": "ARHGAP27"
}